{
  "gene_symbol": "CLCF1",
  "gene_name": "Cardiotrophin-like cytokine factor 1",
  "term_label": "extracellular region",
  "gene": "UniProtKB:Q9UBD9",
  "term_id": "GO:0005576"
}